regulation of cerebral blood circulation [GO:0120276] (biological process) Definition: Any process that modulates the frequency, rate or extent of cerebral blood circulation. References: PMID:25397684 Sources: GOC:krc Also known as: regulation of cerebrum blood circulation, regulation of telencephalon blood circulation Relationships: is a type of regulation of blood circulation [GO:1903522]; regulates cerebral blood circulation [GO:0120275] Subtypes: GO:0120277, GO:0120278